{
  "term_label": "recycling endosome membrane",
  "gene_name": "Secretory carrier-associated membrane protein 1",
  "term_id": "GO:0055038",
  "gene": "UniProtKB:O15126",
  "gene_symbol": "SCAMP1"
}